pronephros maturation [GO:0072120] (biological process) Subtypes: head kidney maturation [GO:0072121] Sources: GOC:mtg_kidney_jan10 Definition: A developmental process, independent of morphogenetic (shape) change, that is required for the pronephros to attain its fully functional state. In mammals, the pronephros is the first of the three embryonic kidneys to be established and exists only transiently. In lower vertebrates such as fish and amphibia, the pronephros is the fully functional embryonic kidney and is indispensable for larval life. Also known as: pronephric kidney maturation Relationships: is a type of GO:0048799; is part of GO:0048793